mannitol catabolic process [GO:0019592] (biological process) Definition: The chemical reactions and pathways resulting in the breakdown of mannitol, the alditol derived from D-mannose by reduction of the aldehyde group. Relationships: is a type of hexitol catabolic process [GO:0019407]; is a type of mannitol metabolic process [GO:0019594] Also known as: mannitol breakdown, mannitol catabolism, mannitol degradation Sources: ISBN:0198506732